{
  "gene_name": "TMF-regulated nuclear protein 1",
  "term_id": "GO:0005634",
  "term_label": "nucleus",
  "gene": "UniProtKB:Q6NT89",
  "gene_symbol": "TRNP1"
}